heparin lyase activity [GO:0047488] (molecular function) Also known as: heparan sulfate lyase activity, heparin eliminase activity, heparinase activity Relationships: is a type of carbon-oxygen lyase activity, acting on polysaccharides [GO:0016837] Definition: Catalysis of the eliminative cleavage of polysaccharides containing 1,4-linked D-glucuronate or L-iduronate residues and 1,4-alpha-linked 2-sulfoamino-2-deoxy-6-sulfo-D-glucose residues to give oligosaccharides with terminal 4-deoxy-alpha-D-gluc-4-enuronosyl groups at their nonreducing ends. Sources: EC:4.2.2.7, MetaCyc:4.2.2.7-RXN